oxylipin metabolic process [GO:0031407] (biological process) Relationships: is a type of carboxylic acid metabolic process [GO:0019752] References: PMID:11960741 Sources: GOC:mah Also known as: oxylipin metabolism Subtypes: oxylipin biosynthetic process [GO:0031408] Definition: The chemical reactions and pathways involving any oxylipin, any of a group of biologically active compounds formed by oxidative metabolism of polyunsaturated fatty acids.